{
  "term_id": "GO:0008017",
  "term_label": "microtubule binding",
  "gene_name": "Microtubule-associated protein 10",
  "gene": "UniProtKB:Q9P2G4",
  "gene_symbol": "MAP10"
}